{
  "gene": "UniProtKB:Q12873",
  "term_id": "GO:0006338",
  "gene_name": "Chromodomain-helicase-DNA-binding protein 3",
  "gene_symbol": "CHD3",
  "term_label": "chromatin remodeling"
}